skeletal muscle tissue development [GO:0007519] (biological process) Sources: GOC:mtg_muscle Subtypes: extraocular skeletal muscle development [GO:0002074], branchiomeric skeletal muscle development [GO:0014707] Also known as: myogenesis Relationships: is a type of GO:0014706; is part of GO:0060538 Definition: The developmental sequence of events leading to the formation of adult skeletal muscle tissue. The main events are: the fusion of myoblasts to form myotubes that increase in size by further fusion to them of myoblasts, the formation of myofibrils within their cytoplasm and the establishment of functional neuromuscular junctions with motor neurons. At this stage they can be regarded as mature muscle fibers. Regulation: regulated by regulation of skeletal muscle tissue development [GO:0048641]; negatively regulated by negative regulation of skeletal muscle tissue development [GO:0048642]; positively regulated by positive regulation of skeletal muscle tissue development [GO:0048643]